{
  "term_label": "Unknown biological process",
  "gene_name": "Pyruvate dehydrogenase phosphatase regulatory subunit, mitochondrial",
  "gene_symbol": "PDPR",
  "term_id": "UNKNOWN:0002",
  "gene": "UniProtKB:Q8NCN5"
}